positive regulation of nuclear mRNA surveillance of meiosis-specific transcripts [GO:0120272] (biological process) Also known as: positive regulation of nuclear-transcribed mRNA catabolic process, meiosis-specific transcripts Definition: Any process that activates or increases the frequency, rate or extent of degradation of meiosis-specific nuclear transcribed transcripts during vegetative growth, by a mechanism that requires determinant of selective removal (DSR) sequences in the targeted mRNAs and involves a YTH family protein. Relationships: is a type of positive regulation of mRNA catabolic process [GO:0061014]; is a type of regulation of nuclear mRNA surveillance of meiosis-specific transcripts [GO:0120270]; positively regulates nuclear mRNA surveillance of meiosis-specific transcripts [GO:0033621] References: PMID:24920274 Sources: GOC:krc